{
  "gene": "UniProtKB:P47895",
  "term_id": "UNKNOWN:0003",
  "term_label": "Unknown cellular component",
  "gene_name": "Retinaldehyde dehydrogenase 3",
  "gene_symbol": "ALDH1A3"
}